ADP-phosphoglycerate phosphatase activity [GO:0047630] (molecular function) Sources: RHEA:15861 Relationships: is_a phosphatase activity [GO:0016791] Also known as: 3-(ADP)-2-phosphoglycerate phosphohydrolase activity, ADPphosphoglycerate phosphatase activity, adenosine diphosphate phosphoglycerate phosphatase activity Definition: Catalysis of the reaction: 3-ADP-2-phosphoglycerate + H2O = 3-ADP-glycerate + phosphate.